H1 histone chaperone activity [GO:0140890] (molecular function) Definition: A histone chaperone that carries a H1 histone. References: PMID:12509435 Also known as: H1 histone carrier activity Relationships: is a type of GO:0140713